{
  "gene": "UniProtKB:Q9Y399",
  "term_id": "GO:0005763",
  "term_label": "mitochondrial small ribosomal subunit",
  "gene_name": "Small ribosomal subunit protein uS2m",
  "gene_symbol": "MRPS2"
}